epithelial cell differentiation [GO:0030855] (biological process) Subtypes: columnar/cuboidal epithelial cell differentiation [GO:0002065], epidermal cell differentiation [GO:0009913], polarized epithelial cell differentiation [GO:0030859], leading edge cell differentiation [GO:0035026], epithelial cell differentiation involved in kidney development [GO:0035850], enteroendocrine cell differentiation [GO:0035883], GO:0045446, Sertoli cell differentiation [GO:0060008], GO:0060014, mesenchymal to epithelial transition [GO:0060231], lung epithelial cell differentiation [GO:0060487], GO:0060644, epithelial cell differentiation involved in embryonic placenta development [GO:0060671], epithelial cell differentiation involved in salivary gland development [GO:0060690], GO:0060742, hepatoblast differentiation [GO:0061017], Malpighian tubule principal cell differentiation [GO:0061329], Malpighian tubule stellate cell differentiation [GO:0061330], GO:0062236, lens fiber cell differentiation [GO:0070306], hepatocyte differentiation [GO:0070365], GO:0072192, GO:0160122 Relationships: is a type of GO:0030154; is part of epithelium development [GO:0060429] References: PMID:11839751 Sources: GOC:ecd Definition: The process in which a relatively unspecialized cell acquires specialized features of an epithelial cell, any of the cells making up an epithelium. Regulation: regulated by regulation of epithelial cell differentiation [GO:0030856]; negatively regulated by negative regulation of epithelial cell differentiation [GO:0030857]; positively regulated by positive regulation of epithelial cell differentiation [GO:0030858]